establishment of protein localization to plasma membrane [GO:0061951] (biological process) Relationships: is a type of establishment of protein localization to membrane [GO:0090150] Definition: The directed movement of a protein to a specific location in a plasma membrane. Subtypes: Golgi to plasma membrane protein transport [GO:0043001], endosome to plasma membrane protein transport [GO:0099638], protein transport from ciliary membrane to plasma membrane [GO:1903445] Sources: GOC:dph, GOC:vw